{
  "gene": "UniProtKB:Q3BBV2",
  "gene_name": "Putative neuroblastoma breakpoint family member 8",
  "term_id": "UNKNOWN:0003",
  "term_label": "Unknown cellular component",
  "gene_symbol": "NBPF8"
}